{
  "gene_name": "Beta-catenin-interacting protein 1",
  "term_label": "nucleus",
  "gene": "UniProtKB:Q9NSA3",
  "gene_symbol": "CTNNBIP1",
  "term_id": "GO:0005634"
}